{
  "gene_name": "Adenylate kinase 4, mitochondrial",
  "term_id": "GO:0046033",
  "gene_symbol": "AK4",
  "gene": "UniProtKB:P27144",
  "term_label": "AMP metabolic process"
}